fibroblast growth factor receptor signaling pathway involved in somitogenesis [GO:0090243] (biological process) Definition: The series of molecular signals generated as a consequence of a fibroblast growth factor receptor binding to one of its physiological ligands that contributes to somitogenesis. Also known as: fibroblast growth factor receptor signalling pathway involved in somitogenesis Relationships: is a type of fibroblast growth factor receptor signaling pathway [GO:0008543]; is part of GO:0001756 Sources: GOC:ascb_2009, GOC:dph, GOC:tb